{
  "term_id": "GO:0004984",
  "gene_name": "Olfactory receptor 9Q1",
  "gene_symbol": "OR9Q1",
  "gene": "UniProtKB:Q8NGQ5",
  "term_label": "olfactory receptor activity"
}